negative regulation of detection of glucose [GO:2000971] (biological process) Relationships: is a type of negative regulation of response to stimulus [GO:0048585]; is a type of regulation of detection of glucose [GO:2000970]; negatively regulates detection of glucose [GO:0051594] Definition: Any process that stops, prevents or reduces the frequency, rate or extent of detection of glucose. Also known as: negative regulation of glucose detection, negative regulation of glucose perception, negative regulation of glucose sensing Sources: GOC:BHF